{
  "gene": "UniProtKB:O94760",
  "term_id": "GO:0016597",
  "term_label": "amino acid binding",
  "gene_name": "N(G),N(G)-dimethylarginine dimethylaminohydrolase 1",
  "gene_symbol": "DDAH1"
}